{
  "gene": "UniProtKB:O95319",
  "gene_name": "CUGBP Elav-like family member 2",
  "gene_symbol": "CELF2",
  "term_label": "regulation of alternative mRNA splicing, via spliceosome",
  "term_id": "GO:0000381"
}